{
  "term_id": "GO:0006357",
  "gene_symbol": "ZNF283",
  "gene": "UniProtKB:Q8N7M2",
  "term_label": "regulation of transcription by RNA polymerase II",
  "gene_name": "Zinc finger protein 283"
}